Golgi localization [GO:0051645] (biological process) Definition: Any process in which the Golgi is transported to, and/or maintained in, a specific location within the cell. Subtypes: establishment of Golgi localization [GO:0051683], maintenance of Golgi location [GO:0051684], Golgi distribution to daughter cells [GO:0090167] Relationships: is a type of GO:0051640 Also known as: Golgi apparatus localization, Golgi body localization, Golgi localisation, establishment and maintenance of Golgi localization Sources: GOC:ai